regulation of neutrophil apoptotic process [GO:0033029] (biological process) Definition: Any process that modulates the frequency, rate, or extent of neutrophil apoptotic process. Also known as: regulation of neutrophil apoptosis Subtypes: negative regulation of neutrophil apoptotic process [GO:0033030], positive regulation of neutrophil apoptotic process [GO:0033031] Sources: GOC:add, GOC:mtg_apoptosis Relationships: is a type of regulation of immune system process [GO:0002682]; is a type of regulation of myeloid cell apoptotic process [GO:0033032]; is a type of GO:2000106; regulates GO:0001781